{
  "gene": "UniProtKB:Q9NPG2",
  "gene_symbol": "NGB",
  "gene_name": "Neuroglobin",
  "term_label": "oxygen carrier activity",
  "term_id": "GO:0005344"
}